{
  "term_id": "UNKNOWN:0002",
  "term_label": "Unknown biological process",
  "gene_name": "FK506-binding protein-like",
  "gene_symbol": "FKBPL",
  "gene": "UniProtKB:Q9UIM3"
}